dibenzo-p-dioxin metabolic process [GO:0018894] (biological process) Also known as: dibenzo-p-dioxin metabolism, oxanthrene metabolic process, oxanthrene metabolism, phenodioxin metabolic process, phenodioxin metabolism Subtypes: dibenzo-p-dioxin catabolic process [GO:0019341] Sources: UM-BBD_pathwayID:dpd Relationships: is a type of GO:0044281 Definition: The chemical reactions and pathways involving dibenzo-p-dioxin, a substance composed of two benzene rings linked by two ether bonds. Dibenzo-p-dioxins are generated as by-products in the manufacturing of herbicides, insecticides, fungicides, paper pulp bleaching, and in incineration, and can accumulate in milk and throughout the food chain, creating significant health concern.